positive regulation of lymphocyte mediated immunity [GO:0002708] (biological process) Also known as: up regulation of lymphocyte mediated immunity, up-regulation of lymphocyte mediated immunity, upregulation of lymphocyte mediated immunity, activation of lymphocyte mediated immunity, stimulation of lymphocyte mediated immunity Subtypes: positive regulation of T cell mediated immunity [GO:0002711], positive regulation of B cell mediated immunity [GO:0002714], positive regulation of natural killer cell mediated immunity [GO:0002717] Sources: GOC:add Definition: Any process that activates or increases the frequency, rate, or extent of lymphocyte mediated immunity. Relationships: is a type of GO:0002705; is a type of regulation of lymphocyte mediated immunity [GO:0002706]; positively regulates lymphocyte mediated immunity [GO:0002449]